carbon catabolite repression of transcription from RNA polymerase II promoter by galactose [GO:0000434] (biological process) Definition: Any process involving galactose that stops, prevents or reduces the rate of transcription from an RNA polymerase II promoter. Relationships: is a type of carbon catabolite repression of transcription by galactose [GO:0000410]; is a type of GO:0000431; is a type of carbon catabolite repression of transcription from RNA polymerase II promoter [GO:0000437] Sources: GOC:krc Also known as: down regulation of transcription from RNA polymerase II promoter by galactose, down-regulation of transcription from RNA polymerase II promoter by galactose, downregulation of transcription from RNA polymerase II promoter by galactose, inhibition of transcription from RNA polymerase II promoter by galactose